{
  "gene": "UniProtKB:Q6PII3",
  "term_id": "UNKNOWN:0002",
  "gene_name": "Coiled-coil domain-containing protein 174",
  "term_label": "Unknown biological process",
  "gene_symbol": "CCDC174"
}